{
  "gene_symbol": "ESYT3",
  "term_id": "GO:0005509",
  "gene_name": "Extended synaptotagmin-3",
  "gene": "UniProtKB:A0FGR9",
  "term_label": "calcium ion binding"
}